{
  "gene": "UniProtKB:P0C7M6",
  "gene_name": "IQ domain-containing protein F3",
  "term_label": "Unknown biological process",
  "gene_symbol": "IQCF3",
  "term_id": "UNKNOWN:0002"
}